{
  "gene": "UniProtKB:Q9HA64",
  "term_label": "kinase activity",
  "term_id": "GO:0016301",
  "gene_symbol": "FN3KRP",
  "gene_name": "Ketosamine-3-kinase"
}